striated muscle dense body [GO:0055120] (cellular component) Definition: A vinculin-containing myofibril attachment structure of striated muscle that connects sarcomeres to the extracellular matrix. In nematode body wall muscle, the dense body performs the dual role of Z-disk and costamere. Relationships: is a type of cellular anatomical structure [GO:0110165]; BFO_0000050 GO:0043292 References: PMID:17492481 Sources: GOC:kmv